{
  "term_label": "Unknown biological process",
  "gene_symbol": "CACNA2D1",
  "gene": "UniProtKB:P54289",
  "term_id": "UNKNOWN:0002",
  "gene_name": "Voltage-dependent calcium channel subunit alpha-2_delta-1"
}